{
  "gene_symbol": "CPAMD8",
  "term_id": "UNKNOWN:0003",
  "term_label": "Unknown cellular component",
  "gene": "UniProtKB:Q8IZJ3",
  "gene_name": "C3 and PZP-like alpha-2-macroglobulin domain-containing protein 8"
}